{
  "term_label": "vesicle-mediated transport",
  "gene": "UniProtKB:Q9NYI0",
  "gene_name": "PH and SEC7 domain-containing protein 3",
  "term_id": "GO:0016192",
  "gene_symbol": "PSD3"
}